{
  "gene_name": "Olfactory receptor 1I1",
  "gene_symbol": "OR1I1",
  "term_label": "signal transduction",
  "term_id": "GO:0007165",
  "gene": "UniProtKB:O60431"
}